response to muramyl dipeptide [GO:0032495] (biological process) Definition: Any process that results in a change in state or activity of an organism (in terms of movement, secretion, enzyme production, gene expression, etc.) as a result of a muramyl dipeptide stimulus. Muramyl dipeptide is derived from peptidoglycan. Relationships: is a type of response to nitrogen compound [GO:1901698]; is a type of response to oxygen-containing compound [GO:1901700] Sources: GOC:add Subtypes: detection of muramyl dipeptide [GO:0032498], GO:0071225